{
  "term_label": "cytoplasm",
  "gene_symbol": "ZMYND8",
  "gene": "UniProtKB:Q9ULU4",
  "term_id": "GO:0005737",
  "gene_name": "MYND-type zinc finger-containing chromatin reader ZMYND8"
}